{
  "term_id": "UNKNOWN:0002",
  "gene_name": "Cyclin-dependent kinase 19",
  "gene_symbol": "CDK19",
  "gene": "UniProtKB:Q9BWU1",
  "term_label": "Unknown biological process"
}